{
  "term_id": "GO:0006357",
  "gene": "UniProtKB:Q7L2R6",
  "gene_symbol": "ZNF765",
  "gene_name": "Zinc finger protein 765",
  "term_label": "regulation of transcription by RNA polymerase II"
}